{
  "gene_name": "Sperm flagellar protein 2",
  "term_id": "GO:0002177",
  "gene": "UniProtKB:Q9C093",
  "term_label": "manchette",
  "gene_symbol": "SPEF2"
}